{
  "gene_symbol": "USP8",
  "gene": "UniProtKB:P40818",
  "term_id": "GO:0004843",
  "gene_name": "Ubiquitin carboxyl-terminal hydrolase 8",
  "term_label": "cysteine-type deubiquitinase activity"
}